{
  "term_id": "GO:0005886",
  "term_label": "plasma membrane",
  "gene": "UniProtKB:Q96S21",
  "gene_name": "Ras-related protein Rab-40C",
  "gene_symbol": "RAB40C"
}